{
  "gene_name": "Protein unc-119 homolog B",
  "gene": "UniProtKB:A6NIH7",
  "gene_symbol": "UNC119B",
  "term_label": "nervous system development",
  "term_id": "GO:0007399"
}